{
  "gene": "UniProtKB:O00757",
  "term_label": "gluconeogenesis",
  "gene_name": "Fructose-1,6-bisphosphatase isozyme 2",
  "term_id": "GO:0006094",
  "gene_symbol": "FBP2"
}